{
  "term_id": "GO:0140375",
  "term_label": "immune receptor activity",
  "gene_symbol": "KIR2DP1",
  "gene": "UniProtKB:A0A0G2JNF4",
  "gene_name": "Killer cell immunoglobulin-like receptor, two Ig domains pseudogene 1"
}